{
  "gene_symbol": "MED1",
  "term_label": "nuclear retinoic acid receptor binding",
  "term_id": "GO:0042974",
  "gene_name": "Mediator of RNA polymerase II transcription subunit 1",
  "gene": "UniProtKB:Q15648"
}